{
  "gene": "UniProtKB:Q8IV16",
  "term_id": "GO:0005886",
  "gene_name": "Glycosylphosphatidylinositol-anchored high density lipoprotein-binding protein 1",
  "gene_symbol": "GPIHBP1",
  "term_label": "plasma membrane"
}